{
  "term_label": "organelle fusion",
  "gene_name": "Vacuolar protein sorting-associated protein 18 homolog",
  "term_id": "GO:0048284",
  "gene_symbol": "VPS18",
  "gene": "UniProtKB:Q9P253"
}